{
  "gene_name": "PDZ and LIM domain protein 3",
  "term_label": "actin cytoskeleton organization",
  "gene": "UniProtKB:Q53GG5",
  "gene_symbol": "PDLIM3",
  "term_id": "GO:0030036"
}